{
  "gene_name": "Tubulin beta-4B chain",
  "term_label": "structural constituent of cytoskeleton",
  "term_id": "GO:0005200",
  "gene_symbol": "TUBB4B",
  "gene": "UniProtKB:P68371"
}